{
  "term_id": "GO:0051899",
  "gene": "UniProtKB:Q04844",
  "gene_name": "Acetylcholine receptor subunit epsilon",
  "term_label": "membrane depolarization",
  "gene_symbol": "CHRNE"
}